{
  "gene_symbol": "P2RX4",
  "term_label": "extracellularly ATP-gated monoatomic cation channel activity",
  "gene_name": "P2X purinoceptor 4",
  "gene": "UniProtKB:Q99571",
  "term_id": "GO:0004931"
}